regulation of penicillin catabolic process [GO:0033247] (biological process) Sources: GOC:mah Definition: Any process that modulates the frequency, rate or extent of the chemical reactions and pathways leading to the breakdown of any antibiotic that contains the condensed beta-lactamthiazolidine ring system. Relationships: is a type of regulation of catabolic process [GO:0009894]; is a type of GO:0034248; is a type of regulation of sulfur metabolic process [GO:0042762]; is a type of regulation of secondary metabolic process [GO:0043455]; is a type of regulation of small molecule metabolic process [GO:0062012]; regulates penicillin catabolic process [GO:0042317] Also known as: regulation of penicillin breakdown, regulation of penicillin catabolism, regulation of penicillin degradation Subtypes: negative regulation of penicillin catabolic process [GO:0033248], positive regulation of penicillin catabolic process [GO:0033249]